{
  "term_label": "plasma membrane",
  "gene_symbol": "MRC1",
  "gene_name": "Macrophage mannose receptor 1",
  "term_id": "GO:0005886",
  "gene": "UniProtKB:P22897"
}